{
  "term_label": "plasma membrane",
  "gene_name": "Ankyrin repeat domain-containing protein 27",
  "term_id": "GO:0005886",
  "gene_symbol": "ANKRD27",
  "gene": "UniProtKB:Q96NW4"
}